negative regulation of corticosteroid hormone secretion [GO:2000847] (biological process) Subtypes: negative regulation of glucocorticoid secretion [GO:2000850], negative regulation of mineralocorticoid secretion [GO:2000856] Relationships: is a type of GO:2000832; is_a regulation of corticosteroid hormone secretion [GO:2000846]; negatively regulates corticosteroid hormone secretion [GO:0035930] Also known as: negative regulation of corticosteroid secretion Definition: Any process that stops, prevents or reduces the frequency, rate or extent of corticosteroid hormone secretion. Sources: GOC:sl